{
  "gene_symbol": "CECR9",
  "term_id": "UNKNOWN:0001",
  "term_label": "Unknown molecular function",
  "gene": "UniProtKB:P0C854",
  "gene_name": "Putative cat eye syndrome critical region protein 9"
}